cerebellum structural organization [GO:0021589] (biological process) Definition: The process that contributes to the act of creating the structural organization of the cerebellum. This process pertains to the physical shaping of a rudimentary structure. The cerebellum is the portion of the brain in the back of the head between the cerebrum and the pons. The cerebellum controls balance for walking and standing, modulates the force and range of movement and is involved in the learning of motor skills. Sources: GOC:cls, GOC:dgh, GOC:dph, GOC:jid, GO_REF:0000021 Also known as: cerebellum structural organisation Relationships: is_a anatomical structure arrangement [GO:0048532]; is part of hindbrain structural organization [GO:0021577]; is part of cerebellum morphogenesis [GO:0021587]